{
  "term_label": "phosphatidylserine floppase activity",
  "gene_name": "Phospholipid-transporting ATPase ABCA7",
  "gene_symbol": "ABCA7",
  "term_id": "GO:0090556",
  "gene": "UniProtKB:Q8IZY2"
}